carbohydrate import across plasma membrane [GO:0098704] (biological process) Also known as: carbohydrate import into cell Definition: The directed movement of a carbohydrate from outside of a cell, across the plasma membrane and into the cytosol. Relationships: is_a carbohydrate transmembrane transport [GO:0034219]; is a type of import across plasma membrane [GO:0098739] Sources: GOC:dos Subtypes: phosphoenolpyruvate-dependent sugar phosphotransferase system [GO:0009401], maltose import across plasma membrane [GO:0106081], sucrose import across plasma membrane [GO:0106082], hexose import across plasma membrane [GO:0140271]